{
  "gene_name": "Proline-rich protein 13",
  "gene": "UniProtKB:Q9NZ81",
  "term_id": "UNKNOWN:0001",
  "gene_symbol": "PRR13",
  "term_label": "Unknown molecular function"
}